mandelate catabolic process [GO:0019596] (biological process) Relationships: is a type of mandelate metabolic process [GO:0018924]; is a type of GO:0072329 Sources: GOC:go_curators Also known as: mandelate breakdown, mandelate catabolism, mandelate degradation Definition: The chemical reactions and pathways resulting in the breakdown of mandelate, the anion of mandelic acid. Mandelic acid (alpha-hydroxybenzeneacetic acid) is an 8-carbon alpha-hydroxy acid (AHA) that is used in organic chemistry and as a urinary antiseptic. Subtypes: (R)-mandelate catabolic process to benzoate [GO:0019597], (R)-mandelate catabolic process to catechol [GO:0019598]